{
  "gene_name": "Outer dense fiber protein 1",
  "term_label": "Unknown biological process",
  "term_id": "UNKNOWN:0002",
  "gene_symbol": "ODF1",
  "gene": "UniProtKB:Q14990"
}